{
  "term_label": "Unknown cellular component",
  "gene_symbol": "JKAMP",
  "gene": "UniProtKB:Q9P055",
  "term_id": "UNKNOWN:0003",
  "gene_name": "JNK1_MAPK8-associated membrane protein"
}